early endosome to Golgi transport [GO:0034498] (biological process) Relationships: is a type of retrograde transport, endosome to Golgi [GO:0042147]; is a type of Golgi vesicle transport [GO:0048193] Sources: GOC:rb Definition: The directed movement of substances from early endosomes to the Golgi. Also known as: PGE to Golgi transport, post-Golgi endosome to Golgi transport